{
  "term_label": "semaphorin receptor complex",
  "gene_symbol": "PLXNB1",
  "gene": "UniProtKB:O43157",
  "gene_name": "Plexin-B1",
  "term_id": "GO:0002116"
}